dipeptide uniporter activity [GO:0160178] (molecular function) Definition: Catalysis of the transport of a dipeptide across a membrane; transport is independent of the movement of any other molecular species. Relationships: is a type of GO:0015292; is a type of dipeptide transmembrane transporter activity [GO:0071916] References: PMID:38507452